alpha9-beta1 integrin-thrombospondin-1 complex [GO:0071134] (cellular component) Also known as: ITGA9-ITGB1-THBS1 complex References: PMID:17413041 Definition: A protein complex that consists of an alpha9-beta1 integrin complex bound to thrombospondin-1. Relationships: is a type of plasma membrane protein complex [GO:0098797]